{
  "term_label": "regulation of axonogenesis",
  "term_id": "GO:0050770",
  "gene": "UniProtKB:Q13177",
  "gene_symbol": "PAK2",
  "gene_name": "Serine_threonine-protein kinase PAK 2"
}